{
  "gene_symbol": "TM4SF1",
  "gene_name": "Transmembrane 4 L6 family member 1",
  "term_label": "Unknown biological process",
  "gene": "UniProtKB:P30408",
  "term_id": "UNKNOWN:0002"
}